dAMP biosynthetic process [GO:0006170] (biological process) Relationships: is a type of purine deoxyribonucleotide biosynthetic process [GO:0009153]; is a type of GO:0009171; is a type of dAMP metabolic process [GO:0046053] Subtypes: dAMP salvage [GO:0106383] Sources: ISBN:0198506732 Definition: The chemical reactions and pathways resulting in the formation of dAMP, deoxyadenosine monophosphate (2'-deoxyadenosine 5'-phosphate). Also known as: dAMP anabolism, dAMP biosynthesis, dAMP formation, dAMP synthesis